{
  "gene_symbol": "CRYM",
  "gene": "UniProtKB:Q14894",
  "term_id": "GO:0070324",
  "gene_name": "Ketimine reductase mu-crystallin",
  "term_label": "thyroid hormone binding"
}